{
  "term_label": "transcription elongation factor complex",
  "gene": "UniProtKB:Q03111",
  "gene_name": "Protein ENL",
  "gene_symbol": "MLLT1",
  "term_id": "GO:0008023"
}